antisense RNA metabolic process [GO:0042868] (BP) Subtypes: GO:0009300, antisense RNA transcript catabolic process [GO:0071041] Definition: The chemical reactions and pathways involving antisense RNA, an RNA molecule complementary in sequence to another RNA or DNA molecule, which, by binding the latter, acts to inhibit its function and/or completion of synthesis. Relationships: is a type of RNA metabolic process [GO:0016070] Also known as: antisense RNA metabolism Sources: GOC:jl